{
  "gene_name": "2'-5'-oligoadenylate synthase 2",
  "term_label": "cytosol",
  "term_id": "GO:0005829",
  "gene_symbol": "OAS2",
  "gene": "UniProtKB:P29728"
}